{
  "gene": "UniProtKB:P57060",
  "gene_symbol": "RWDD2B",
  "term_id": "UNKNOWN:0001",
  "gene_name": "RWD domain-containing protein 2B",
  "term_label": "Unknown molecular function"
}